galactonate catabolic process [GO:0019584] (BP) Definition: The chemical reactions and pathways resulting in the breakdown of galactonate, the anion of galactonic acid. Subtypes: D-galactonate catabolic process [GO:0034194], L-galactonate catabolic process [GO:0034195] Relationships: is a type of aldonic acid catabolic process [GO:0046176] Also known as: galactonate breakdown, galactonate catabolism, galactonate degradation Sources: GOC:ai